terminal branching, open tracheal system [GO:0007430] (biological process) Also known as: terminal branching of trachea, cytoplasmic projection extension References: PMID:29844090 Sources: GOC:mtg_sensu Definition: Formation of terminal branches in the open tracheal system. These are long cytoplasmic extensions that form fine tubules that transport oxygen directly to the tissues. An example of the process is found in Drosophila melanogaster. Relationships: is a type of branching involved in open tracheal system development [GO:0060446]